extracellular ATP signaling [GO:0106167] (biological process) Definition: The series of molecular signals mediated by the detection of extracellular ATP. Relationships: is_a signal transduction [GO:0007165]; is a type of GO:0071318 References: PMID:12948585, PMID:20817461, PMID:29274390 Sources: GOC:tb